{
  "gene_name": "Mitotic spindle assembly checkpoint protein MAD1",
  "gene_symbol": "MAD1L1",
  "term_label": "nuclear envelope",
  "term_id": "GO:0005635",
  "gene": "UniProtKB:Q9Y6D9"
}